lupeol synthase activity [GO:0042299] (molecular function) Relationships: is a type of GO:0031559 References: PMID:9883589 Sources: MetaCyc:RXN-111 Also known as: oxidosqualene:lupeol cyclase activity Definition: Catalysis of the reaction: (S)-2,3-epoxysqualene = lupeol. This reaction is the cyclization of (S)-2,3-epoxysqualene (2,3-oxidosqualene) to lupeol.